metanephric cortex development [GO:0072214] (BP) Sources: GOC:mtg_kidney_jan10 Definition: The process whose specific outcome is the progression of the metanephric cortex over time, from its formation to the mature structure. The metanephric cortex is the outer region of the metanephros. Relationships: is_a mesenchyme development [GO:0060485]; is a type of renal cortex development [GO:0072055]; is part of metanephros development [GO:0001656]